lymph circulation [GO:0003017] (biological process) Definition: The flow of lymph through the body of an animal. Sources: GOC:mtg_cardio Relationships: is a type of GO:0003013